{
  "gene_symbol": "PLXNA4",
  "term_id": "GO:0017154",
  "term_label": "semaphorin receptor activity",
  "gene_name": "Plexin-A4",
  "gene": "UniProtKB:Q9HCM2"
}